{
  "gene": "UniProtKB:Q9Y5J9",
  "term_id": "UNKNOWN:0003",
  "gene_name": "Mitochondrial import inner membrane translocase subunit Tim8 B",
  "term_label": "Unknown cellular component",
  "gene_symbol": "TIMM8B"
}